{
  "term_label": "alanine-glyoxylate transaminase activity",
  "term_id": "GO:0008453",
  "gene": "UniProtKB:Q9BYV1",
  "gene_name": "Alanine--glyoxylate aminotransferase 2, mitochondrial",
  "gene_symbol": "AGXT2"
}